{
  "gene_symbol": "TXNDC8",
  "gene": "UniProtKB:Q6A555",
  "term_id": "UNKNOWN:0001",
  "gene_name": "Thioredoxin domain-containing protein 8",
  "term_label": "Unknown molecular function"
}